{
  "term_label": "leukocyte migration",
  "gene_symbol": "ITGB7",
  "gene": "UniProtKB:P26010",
  "gene_name": "Integrin beta-7",
  "term_id": "GO:0050900"
}